{
  "gene_symbol": "ZNF579",
  "gene": "UniProtKB:Q8NAF0",
  "gene_name": "Zinc finger protein 579",
  "term_id": "UNKNOWN:0001",
  "term_label": "Unknown molecular function"
}